RNA uridylyltransferase activity [GO:0050265] (molecular function) Sources: EC:2.7.7.52, MetaCyc:RNA-URIDYLYLTRANSFERASE-RXN Relationships: is_a GO:0070569; is a type of catalytic activity, acting on RNA [GO:0140098] Also known as: UTP:RNA uridylyltransferase activity, poly(U) polymerase activity, polynucleotide uridylyltransferase activity, TUT activity, terminal uridylyltransferase activity Definition: Catalysis of the reaction: UTP + RNA(n) = diphosphate + RNA(n+1).